{
  "term_label": "plasma membrane",
  "gene": "UniProtKB:Q0JRZ9",
  "term_id": "GO:0005886",
  "gene_name": "F-BAR domain only protein 2",
  "gene_symbol": "FCHO2"
}